dTTP diphosphatase activity [GO:0036218] (molecular function) Relationships: is a type of nucleoside triphosphate diphosphatase activity [GO:0047429] Also known as: dTTP pyrophosphatase activity Definition: Catalysis of the reaction: dTTP + H2O = dTMP + H+ + diphosphate. References: PMID:22531138 Sources: GOC:dgf, RHEA:28534